proteoglycan metabolic process [GO:0006029] (BP) Also known as: proteoglycan metabolism, proteoglycan sulfate transfer Definition: The chemical reactions and pathways involving proteoglycans, any glycoprotein in which the carbohydrate units are glycosaminoglycans. Subtypes: cell wall proteoglycan metabolic process [GO:0010384], proteoglycan biosynthetic process [GO:0030166], proteoglycan catabolic process [GO:0030167], GO:0030201, heparin proteoglycan metabolic process [GO:0030202], keratan sulfate proteoglycan metabolic process [GO:0042339], chondroitin sulfate proteoglycan metabolic process [GO:0050654], dermatan sulfate proteoglycan metabolic process [GO:0050655] Relationships: is a type of GO:0009100 References: PMID:35536939